{
  "term_label": "cytosol",
  "term_id": "GO:0005829",
  "gene": "UniProtKB:Q14376",
  "gene_symbol": "GALE",
  "gene_name": "UDP-glucose 4-epimerase"
}